negative regulation of filamentous growth [GO:0060258] (biological process) Subtypes: GO:1900429 Definition: Any process that decreases the frequency, rate or extent of the process in which a multicellular organism or a group of unicellular organisms grow in a threadlike, filamentous shape. Relationships: is_a regulation of filamentous growth [GO:0010570]; is a type of negative regulation of growth [GO:0045926]; negatively regulates filamentous growth [GO:0030447] Sources: GOC:dph, GOC:tb